regulation of nematode larval development, heterochronic [GO:0090444] (biological process) Definition: Any process that modulates the consistent predetermined time point at which a nematode larva progresses from an initial condition to a later condition and the rate at which this time point is reached. References: PMID:17550772 Relationships: is a type of regulation of development, heterochronic [GO:0040034]; is a type of regulation of nematode larval development [GO:0061062] Subtypes: positive regulation of nematode larval development, heterochronic [GO:0090445], negative regulation of nematode larval development, heterochronic [GO:0090446]